positive regulation of eosinophil activation [GO:1902568] (biological process) Relationships: is a type of positive regulation of leukocyte activation [GO:0002696]; is a type of regulation of eosinophil activation [GO:1902566]; positively regulates eosinophil activation [GO:0043307] Definition: Any process that activates or increases the frequency, rate or extent of eosinophil activation. Also known as: up regulation of eosinophil activation, up-regulation of eosinophil activation, upregulation of eosinophil activation, activation of eosinophil activation References: PMID:16254138 Sources: GOC:TermGenie